single guanine insertion binding [GO:0032142] (molecular function) Relationships: is a type of single base insertion or deletion binding [GO:0032138] Definition: Binding to a double-stranded DNA region containing a single guanine insertion or a deletion that results in an unpaired guanine. Sources: GOC:mah, GOC:vk